{
  "gene_name": "NACHT, LRR and PYD domains-containing protein 3",
  "term_id": "GO:0005737",
  "term_label": "cytoplasm",
  "gene_symbol": "NLRP3",
  "gene": "UniProtKB:Q96P20"
}